response to maltose [GO:0034286] (biological process) Also known as: response to maltose stimulus Definition: Any process that results in a change in state or activity of a cell or an organism (in terms of movement, secretion, enzyme production, gene expression, etc.) as a result of a maltose stimulus. Sources: GOC:sart Subtypes: detection of maltose stimulus [GO:0034289], cellular response to maltose stimulus [GO:0071328] Relationships: is a type of GO:0034285